dimethylsulfoxide oxygenase activity [GO:0103001] (molecular function) Relationships: is a type of GO:0016709 Also known as: assimilatory dimethylsulfide S-monooxygenase activity Definition: Catalysis of the reactions: dimethyl sulfoxide + H+ + NADH + O2 = dimethyl sulfone + H2O + NAD+ and dimethyl sulfide + H+ + NADH + O2 = dimethyl sulfoxide + H2O + NAD+. References: PMID:9345770 Sources: EC:1.14.13.245